UDP-4-keto-6-deoxy-glucose-3,5-epimerase activity [GO:0010489] (molecular function) Relationships: is a type of racemase and epimerase activity, acting on carbohydrates and derivatives [GO:0016857] References: PMID:17190829 Sources: GOC:tair_curators Definition: Catalysis of the reaction: UDP-4-keto-6-deoxyglucose = UDP-4-keto-rhamnose.